{
  "term_label": "protein-macromolecule adaptor activity",
  "gene": "UniProtKB:Q14451",
  "gene_symbol": "GRB7",
  "term_id": "GO:0030674",
  "gene_name": "Growth factor receptor-bound protein 7"
}